{
  "gene_symbol": "RNF216P1",
  "gene_name": "Putative protein RNF216-like",
  "term_id": "UNKNOWN:0001",
  "term_label": "Unknown molecular function",
  "gene": "UniProtKB:Q6NUR6"
}